regulation of neurotransmitter secretion [GO:0046928] (biological process) Sources: GOC:ai Relationships: is_a modulation of chemical synaptic transmission [GO:0050804]; is a type of regulation of neurotransmitter transport [GO:0051588]; is a type of regulation of secretion by cell [GO:1903530]; regulates GO:0007269 Subtypes: positive regulation of neurotransmitter secretion [GO:0001956], regulation of acetylcholine secretion, neurotransmission [GO:0014056], negative regulation of neurotransmitter secretion [GO:0046929], regulation of glutamate secretion, neurotransmission [GO:1903294], regulation of spontaneous neurotransmitter secretion [GO:1904048], regulation of substance P secretion, neurotransmission [GO:1904494], GO:1904624, regulation of synaptic vesicle exocytosis [GO:2000300] Definition: Any process that modulates the frequency, rate or extent of the regulated release of a neurotransmitter from a cell.